{
  "gene": "UniProtKB:O60237",
  "term_id": "GO:0031672",
  "gene_name": "Protein phosphatase 1 regulatory subunit 12B",
  "term_label": "A band",
  "gene_symbol": "PPP1R12B"
}